{
  "term_id": "GO:0005886",
  "gene_symbol": "CNGA2",
  "gene": "UniProtKB:Q16280",
  "term_label": "plasma membrane",
  "gene_name": "Cyclic nucleotide-gated olfactory channel"
}